{
  "gene_name": "Krueppel-like factor 15",
  "gene_symbol": "KLF15",
  "term_label": "nucleus",
  "term_id": "GO:0005634",
  "gene": "UniProtKB:Q9UIH9"
}